{
  "term_id": "GO:0003700",
  "gene": "UniProtKB:Q6ZS27",
  "gene_symbol": "ZNF662",
  "gene_name": "Zinc finger protein 662",
  "term_label": "DNA-binding transcription factor activity"
}